{
  "term_id": "GO:0015630",
  "gene": "UniProtKB:Q96GX5",
  "gene_symbol": "MASTL",
  "gene_name": "Serine_threonine-protein kinase greatwall",
  "term_label": "microtubule cytoskeleton"
}